regulation of endocytosis by exocyst localization [GO:0051600] (biological process) Relationships: is a type of regulation of endocytosis [GO:0030100]; is a type of GO:0051601 Also known as: regulation of endocytosis by exocyst localisation, regulation of site selection of endocytosis, relocation of endocytosis, spatial regulation of endocytosis Sources: GOC:ai, GOC:dph, GOC:tb Definition: Any process in which an exocyst is transported to, or maintained in, a specific location that results in the modulation of endocytosis. An exocyst is a protein complex peripherally associated with the plasma membrane that determines where vesicles dock and fuse.